{
  "gene_name": "Lysosomal proton-coupled steroid conjugate and bile acid symporter SLC46A3",
  "term_label": "transmembrane transporter activity",
  "gene_symbol": "SLC46A3",
  "gene": "UniProtKB:Q7Z3Q1",
  "term_id": "GO:0022857"
}